{
  "term_label": "Unknown biological process",
  "gene_name": "Peptidyl-prolyl cis-trans isomerase FKBP3",
  "term_id": "UNKNOWN:0002",
  "gene_symbol": "FKBP3",
  "gene": "UniProtKB:Q00688"
}